{
  "term_id": "GO:0005524",
  "gene_name": "Putative endoplasmin-like protein",
  "gene": "UniProtKB:Q58FF3",
  "term_label": "ATP binding",
  "gene_symbol": "HSP90B2P"
}